N-benzoyl-4-hydroxyanthranilate 4-O-methyltransferase activity [GO:0030771] (molecular function) Definition: Catalysis of the reaction: N-benzoyl-4-hydroxyanthranilate + S-adenosyl-L-methionine(1+) = N-benzoyl-4-methoxyanthranilate + S-adenosyl-L-homocysteine + H+. Sources: EC:2.1.1.105, RHEA:17405 Also known as: benzoyl-CoA:anthranilate N-benzoyltransferase, N-benzoyl-4-hydroxyanthranilate 4-methyltransferase activity, S-adenosyl-L-methionine:N-benzoyl-4-O-hydroxyanthranilate 4-O-methyltransferase activity Relationships: is a type of GO:0008757